T-tubule [GO:0030315] (cellular component) Definition: Invagination of the plasma membrane of a muscle cell that extends inward from the cell surface around each myofibril. The ends of T-tubules make contact with the sarcoplasmic reticulum membrane. Relationships: is a type of cellular anatomical structure [GO:0110165]; is part of GO:0042383 Sources: GOC:mtg_muscle, ISBN:0815316194 Also known as: transverse tubule, triad